{
  "term_id": "GO:0005634",
  "gene_name": "Ribosomal RNA processing protein 1 homolog A",
  "gene": "UniProtKB:P56182",
  "gene_symbol": "RRP1",
  "term_label": "nucleus"
}